regulation of cytoplasmic microtubule depolymerization [GO:0010937] (biological process) Sources: GOC:dph, GOC:tb Subtypes: negative regulation of axonemal microtubule depolymerization [GO:0007027] Definition: Any process that modulates the frequency, rate or extent of cytoplasmic microtubule depolymerization. Relationships: is a type of regulation of microtubule depolymerization [GO:0031114]; regulates cytoplasmic microtubule depolymerization [GO:0010938]